cell leading edge cell cortex [GO:1904269] (cellular component) Relationships: is a type of cell cortex region [GO:0099738]; is part of cell leading edge [GO:0031252] References: PMID:25843030 Sources: GOC:TermGenie, GOC:kmv, GO_REF:0000064 Also known as: cell cortex of cell leading edge, cell cortex of front of cell, cell cortex of leading edge of cell, cell periphery of cell leading edge, cell periphery of front of cell, cell periphery of leading edge of cell, peripheral cytoplasm of cell leading edge, peripheral cytoplasm of front of cell, peripheral cytoplasm of leading edge of cell Definition: The cell cortex of the leading edge of a cell.